{
  "gene_name": "Pleckstrin homology domain-containing family N member 1",
  "gene_symbol": "PLEKHN1",
  "gene": "UniProtKB:Q494U1",
  "term_id": "GO:0043065",
  "term_label": "positive regulation of apoptotic process"
}